{
  "gene_name": "Pecanex-like protein 2",
  "term_id": "UNKNOWN:0001",
  "gene_symbol": "PCNX2",
  "gene": "UniProtKB:A6NKB5",
  "term_label": "Unknown molecular function"
}